{
  "term_label": "centrosome",
  "gene_name": "Protein JTB",
  "gene_symbol": "JTB",
  "gene": "UniProtKB:O76095",
  "term_id": "GO:0005813"
}